{
  "gene_symbol": "PPP4R2",
  "term_label": "cytoplasm",
  "gene_name": "Serine_threonine-protein phosphatase 4 regulatory subunit 2",
  "term_id": "GO:0005737",
  "gene": "UniProtKB:Q9NY27"
}